{
  "term_id": "GO:0030198",
  "gene_name": "Bone sialoprotein 2",
  "gene": "UniProtKB:P21815",
  "term_label": "extracellular matrix organization",
  "gene_symbol": "IBSP"
}